{
  "term_id": "UNKNOWN:0001",
  "term_label": "Unknown molecular function",
  "gene": "UniProtKB:P0DMW4",
  "gene_symbol": "SMIM10L2A",
  "gene_name": "Small integral membrane protein 10-like protein 2A"
}